positive regulation of cap-independent translational initiation [GO:1903679] (biological process) References: PMID:11959995 Sources: GOC:PARL, GOC:TermGenie, GOC:bf, GO_REF:0000058 Relationships: is a type of GO:1903677; is a type of positive regulation of cytoplasmic translational initiation [GO:1904690]; RO_0002213 cap-independent translational initiation [GO:0002190] Definition: Any process that activates or increases the frequency, rate or extent of cap-independent translational initiation. Also known as: up regulation of cap-independent translational initiation, up-regulation of cap-independent translational initiation, upregulation of cap-independent translational initiation, activation of cap-independent translational initiation